response to tellurium ion [GO:0046690] (biological process) Definition: Any process that results in a change in state or activity of a cell or an organism (in terms of movement, secretion, enzyme production, gene expression, etc.) as a result of a tellurium ion stimulus. Relationships: is a type of response to oxygen-containing compound [GO:1901700] Also known as: response to tellurium, tellurium sensitivity/resistance Subtypes: cellular response to tellurium ion [GO:0071293] Sources: GOC:ai